{
  "term_id": "GO:0005793",
  "gene_symbol": "YIF1A",
  "gene": "UniProtKB:O95070",
  "gene_name": "Protein YIF1A",
  "term_label": "endoplasmic reticulum-Golgi intermediate compartment"
}